{
  "term_label": "proteasome-mediated ubiquitin-dependent protein catabolic process",
  "gene": "UniProtKB:Q6TFL4",
  "gene_symbol": "KLHL24",
  "term_id": "GO:0043161",
  "gene_name": "Kelch-like protein 24"
}